{
  "gene_name": "Src-like-adapter",
  "gene_symbol": "SLA",
  "gene": "UniProtKB:Q13239",
  "term_label": "epidermal growth factor receptor binding",
  "term_id": "GO:0005154"
}